{
  "term_label": "transcription coactivator activity",
  "term_id": "GO:0003713",
  "gene_symbol": "POU2AF1",
  "gene_name": "POU domain class 2-associating factor 1",
  "gene": "UniProtKB:Q16633"
}